anoxia protection [GO:0090519] (biological process) References: PMID:19372430 Sources: GOC:tb Relationships: is a type of response to anoxia [GO:0034059] Definition: Any process in which an organism or cell protects itself from anoxia, which may also result in resistance to repeated exposure to anoxia.